{
  "gene_symbol": "ZNF735",
  "term_label": "DNA-binding transcription factor activity, RNA polymerase II-specific",
  "term_id": "GO:0000981",
  "gene_name": "Putative zinc finger protein 735",
  "gene": "UniProtKB:P0CB33"
}